{
  "term_id": "GO:0000978",
  "gene_name": "Zinc finger and SCAN domain-containing protein 12",
  "term_label": "RNA polymerase II cis-regulatory region sequence-specific DNA binding",
  "gene": "UniProtKB:O43309",
  "gene_symbol": "ZSCAN12"
}